{
  "gene_name": "Protein phosphatase 1 regulatory subunit 15A",
  "gene": "UniProtKB:O75807",
  "gene_symbol": "PPP1R15A",
  "term_id": "GO:0019888",
  "term_label": "protein phosphatase regulator activity"
}